nuclear receptor activity [GO:0004879] (molecular function) Definition: A DNA-binding transcription factor activity regulated by binding to a ligand that modulates the transcription of specific gene sets transcribed by RNA polymerase II. Nuclear receptor ligands are usually lipid-based (such as a steroid hormone) and the binding of the ligand to its receptor often occurs in the cytosol, which leads to its translocation to the nucleus. References: PMID:23457262 Sources: GOC:txnOH-2018 Also known as: RNA polymerase II transcription factor activity, ligand-activated sequence-specific DNA binding, ligand-activated sequence-specific DNA binding RNA polymerase II transcription factor activity, 1,25-(OH)2D3 receptor activity, 9-cis retinoic acid receptor activity, RNA polymerase II transcription factor activity, estrogen-activated sequence-specific DNA binding, RNA polymerase II transcription factor activity, glucocorticoid-activated sequence-specific DNA binding, RXR, androgen receptor activity, calcitriol receptor activity, ecdysteroid hormone receptor activity, estrogen nuclear receptor activity, glucocorticoid receptor activity, juvenile hormone receptor activity, nuclear hormone receptor, retinoic acid receptor activity, retinoid-X receptor activity, thyroid hormone receptor activity, vitamin A receptor activity, vitamin D receptor activity, vitamin D3 receptor activity, ligand-dependent nuclear receptor activity, ligand-dependent transcription factor activity Note: Usage guidance: Nuclear receptors are a protein family defined by the presence of a C4-type zinc finger DNA-binding domain and a ligand binding domain. For nuclear receptors, the DNA binding motif is most often referred to as a response element. GO:0004879 is intended for annotation of nuclear receptors that regulate transcription by binding directly to DNA. Relationships: is a type of GO:0000981; is a type of GO:0038023; is a type of ligand-modulated transcription factor activity [GO:0098531]; is part of GO:0030522 Subtypes: nuclear steroid receptor activity [GO:0003707], bile acid nuclear receptor activity [GO:0038186] Regulation: positively regulated by positive regulation of androgen receptor activity [GO:2000825]